{
  "term_id": "GO:0070840",
  "gene": "UniProtKB:O00399",
  "gene_name": "Dynactin subunit 6",
  "term_label": "dynein complex binding",
  "gene_symbol": "DCTN6"
}